Mrh5C translation activator complex [GO:0180049] (cellular component) References: PMID:34634819, PMID:38499152 Also known as: Mrh5C complex Relationships: is a type of protein-containing complex [GO:0032991] Definition: A protein complex capable of translation activator activity, and is involved in the activation of cox1 mRNA for translation. In fission yeast this complex consists of a scaffold (Sls1), a helicase (Mrh5), and PPR repeat proteins Prr4 and Mtf2.